negative regulation of lymphocyte apoptotic process [GO:0070229] (biological process) Subtypes: GO:0002903, negative regulation of T cell apoptotic process [GO:0070233], negative regulation of natural killer cell apoptotic process [GO:0070248] Note: Note that a lymphocyte is a cell of the B cell, T cell, or natural killer cell lineage (CL:0000542). Relationships: is a type of regulation of lymphocyte apoptotic process [GO:0070228]; is a type of GO:2000107; negatively regulates lymphocyte apoptotic process [GO:0070227] Sources: GOC:add, GOC:mtg_apoptosis, ISBN:0781765196 Definition: Any process that stops, prevents, or reduces the frequency, rate or extent of lymphocyte death by apoptotic process. Also known as: down regulation of lymphocyte apoptosis, down-regulation of lymphocyte apoptosis, downregulation of lymphocyte apoptosis, inhibition of lymphocyte apoptosis, negative regulation of lymphocyte apoptosis